{
  "gene": "UniProtKB:P0CJ79",
  "gene_symbol": "ZNF888",
  "term_label": "DNA-binding transcription factor activity, RNA polymerase II-specific",
  "gene_name": "Zinc finger protein 888",
  "term_id": "GO:0000981"
}